{
  "term_label": "plasma membrane",
  "term_id": "GO:0005886",
  "gene_symbol": "KCNJ12",
  "gene_name": "ATP-sensitive inward rectifier potassium channel 12",
  "gene": "UniProtKB:Q14500"
}